{
  "term_id": "UNKNOWN:0003",
  "gene_name": "Pleckstrin homology-like domain family B member 3",
  "gene": "UniProtKB:Q6NSJ2",
  "gene_symbol": "PHLDB3",
  "term_label": "Unknown cellular component"
}